{
  "gene": "UniProtKB:Q9ULB1",
  "term_id": "GO:0007612",
  "term_label": "learning",
  "gene_symbol": "NRXN1",
  "gene_name": "Neurexin-1"
}